{
  "term_id": "UNKNOWN:0001",
  "gene_symbol": "EPB41L2",
  "term_label": "Unknown molecular function",
  "gene": "UniProtKB:O43491",
  "gene_name": "Band 4.1-like protein 2"
}